secondary growth [GO:0080117] (biological process) Regulation: regulated by regulation of secondary growth [GO:2000603]; negatively regulated by negative regulation of secondary growth [GO:2000604]; positively regulated by positive regulation of secondary growth [GO:2000605] Relationships: is a type of lateral growth [GO:0080190] Also known as: cambial secondary growth Note: Occurs in vascular plants, including gymnosperms and most dicotyledons. Commonly supplemented by activity of the cork cambium or phellogen (PO:0005599). Monocotyledons do not have secondary growth, but may undergo primary thickening (GO:0080192) or secondary thickening (GO:0080191), which can give the appearance of secondary growth. Primary and secondary growth can occur simultaneously in the same organism. References: PMID:19074290 Sources: ISBN:0471245208, PO:0005598, PO:0025004 Definition: Lateral growth of a plant axis (shoot axis or root) that is an increase in thickness resulting from formation of secondary vascular tissues by the vascular cambium.